{
  "term_id": "GO:0004467",
  "term_label": "long-chain fatty acid-CoA ligase activity",
  "gene_symbol": "SLC27A6",
  "gene_name": "Long-chain fatty acid transport protein 6",
  "gene": "UniProtKB:Q9Y2P4"
}